{
  "gene_name": "Four and a half LIM domains protein 5",
  "gene": "UniProtKB:Q5TD97",
  "term_label": "Z disc",
  "gene_symbol": "FHL5",
  "term_id": "GO:0030018"
}